{
  "term_id": "GO:0005829",
  "gene_symbol": "NADK",
  "term_label": "cytosol",
  "gene_name": "NAD kinase",
  "gene": "UniProtKB:O95544"
}